{
  "gene_name": "Polypeptide N-acetylgalactosaminyltransferase 4",
  "gene": "UniProtKB:Q8N4A0",
  "gene_symbol": "GALNT4",
  "term_label": "polypeptide N-acetylgalactosaminyltransferase activity",
  "term_id": "GO:0004653"
}